{
  "term_label": "cytoplasm",
  "gene_symbol": "VPS4A",
  "term_id": "GO:0005737",
  "gene_name": "Vacuolar protein sorting-associated protein 4A",
  "gene": "UniProtKB:Q9UN37"
}